UDP-N-acetylgalactosamine transmembrane transporter activity [GO:0005463] (molecular function) Definition: Enables the transfer of a N-acetylgalactosamine from one side of a membrane to the other. N-acetylgalactosamine is a substance composed of N-acetylgalactosamine, a common structural unit of oligosaccharides, in glycosidic linkage with uridine diphosphate. Relationships: is_a pyrimidine nucleotide-sugar transmembrane transporter activity [GO:0015165]; is part of UDP-N-acetylgalactosamine transmembrane transport [GO:0015789] Sources: GOC:ai, GOC:mtg_transport, ISBN:0815340729